{
  "gene_symbol": "ACAA1",
  "term_id": "GO:0005777",
  "gene": "UniProtKB:P09110",
  "term_label": "peroxisome",
  "gene_name": "3-ketoacyl-CoA thiolase, peroxisomal"
}